{
  "gene": "UniProtKB:Q9Y6U3",
  "gene_symbol": "SCIN",
  "term_label": "barbed-end actin filament capping",
  "gene_name": "Scinderin",
  "term_id": "GO:0051016"
}